{
  "gene_symbol": "H4C16",
  "term_label": "nucleosome assembly",
  "gene_name": "Histone H4",
  "gene": "UniProtKB:P62805",
  "term_id": "GO:0006334"
}